cytochrome-b5 reductase activity, acting on NADH [GO:0090524] (molecular function) Also known as: cytochrome b5 reductase activity, NADH 5alpha-reductase activity, NADH-cytochrome b5 reductase activity, NADH-cytochrome-b5 reductase activity, NADH-ferricytochrome b5 oxidoreductase activity, NADH:ferricytochrome-b5 oxidoreductase activity, dihydronicotinamide adenine dinucleotide-cytochrome b5 reductase activity, reduced nicotinamide adeninedinucleotide-cytochrome b5 reductase activity Sources: RHEA:46680 Relationships: is a type of cytochrome-b5 reductase activity, acting on NAD(P)H [GO:0004128] Definition: Catalysis of the reaction: 2 Fe(III)-[cytochrome b5] + NADH = 2 Fe(II)-[cytochrome b5] + NAD+ + H+.